reduced coenzyme F420 dehydrogenase activity [GO:0043738] (molecular function) Sources: RHEA:54752 Definition: Catalysis of the reaction: methanophenazine + reduced coenzyme F420 = dihydromethanophenazine + coenzyme F420. Relationships: is a type of oxidoreductase activity, acting on the CH-NH group of donors [GO:0016645] Also known as: 1,5-dihydrocoenzyme F420 dehydrogenase activity, F420H2 dehydrogenase activity